{
  "gene": "UniProtKB:Q8WU66",
  "gene_name": "Thrombospondin-type laminin G domain and EAR repeat-containing protein",
  "gene_symbol": "TSPEAR",
  "term_id": "UNKNOWN:0001",
  "term_label": "Unknown molecular function"
}